{
  "term_label": "guanyl-nucleotide exchange factor activity",
  "gene": "UniProtKB:Q92902",
  "gene_symbol": "HPS1",
  "term_id": "GO:0005085",
  "gene_name": "BLOC-3 complex member HPS1"
}